{
  "gene_symbol": "FCN3",
  "gene_name": "Ficolin-3",
  "gene": "UniProtKB:O75636",
  "term_label": "complement activation, lectin pathway",
  "term_id": "GO:0001867"
}